regulation of COPII vesicle uncoating [GO:0090111] (biological process) Sources: GOC:ascb_2009, GOC:dph, GOC:tb Relationships: is a type of regulation of protein depolymerization [GO:1901879]; regulates COPII vesicle uncoating [GO:0090112] Definition: Any process that modulates the frequency, rate or extent of COPII vesicle uncoating, the process in which COPII vesicle coat proteins are disassembled, and released.